{
  "gene_name": "Zinc finger protein ZIC 3",
  "term_id": "GO:0045944",
  "gene_symbol": "ZIC3",
  "gene": "UniProtKB:O60481",
  "term_label": "positive regulation of transcription by RNA polymerase II"
}